{
  "term_label": "cell cortex",
  "gene_symbol": "NLRP5",
  "term_id": "GO:0005938",
  "gene_name": "NACHT, LRR and PYD domains-containing protein 5",
  "gene": "UniProtKB:P59047"
}